pyrroline-5-carboxylate reductase activity [GO:0004735] (molecular function) Definition: Catalysis of the reaction: L-proline + NADP+ = 1-pyrroline-5-carboxylate + NADPH + H+. Sources: EC:1.5.1.2 Also known as: 1-pyrroline-5-carboxylate reductase activity, L-proline oxidase activity, L-proline-NAD(P)+ 5-oxidoreductase activity, L-proline:NAD(P)+ 5-oxidoreductase activity, NADPH-L-delta1-pyrroline carboxylic acid reductase activity, P5CR activity Relationships: is a type of GO:0016646